nuclear proteasome complex [GO:0031595] (cellular component) Definition: A proteasome found in the nucleus of a cell. Sources: GOC:mah Relationships: is a type of GO:0000502; is a type of nuclear protein-containing complex [GO:0140513]; is part of GO:0031981